{
  "term_id": "UNKNOWN:0002",
  "gene": "UniProtKB:Q9BRJ7",
  "term_label": "Unknown biological process",
  "gene_symbol": "NUDT16L1",
  "gene_name": "Tudor-interacting repair regulator protein"
}